armadillo repeat domain binding [GO:0070016] (molecular function) Relationships: is a type of GO:0019904 Definition: Binding to an armadillo repeat domain, an approximately 40 amino acid long tandemly repeated sequence motif first identified in the Drosophila segment polarity protein armadillo. Arm-repeat proteins are involved in various processes, including intracellular signaling and cytoskeletal regulation. Also known as: Arm repeat domain binding, armadillo domain binding, armadillo repeat binding Sources: GOC:BHF, GOC:mah, GOC:vk, InterPro:IPR000225